zinc ion import into zymogen granule [GO:0140915] (biological process) Definition: The directed import of zinc(2+) from the cytosol, across an organelle membrane, into a zymogen granule. Relationships: is a type of GO:0140914 References: PMID:20133611